{
  "gene_symbol": "AGER",
  "gene_name": "Advanced glycosylation end product-specific receptor",
  "term_label": "plasma membrane",
  "gene": "UniProtKB:Q15109",
  "term_id": "GO:0005886"
}